pattern recognition receptor activity [GO:0038187] (molecular function) Sources: GOC:ar, GOC:bf Relationships: is a type of signaling receptor activity [GO:0038023] Also known as: PRR, PRR activity, MAMP receptor activity, PAMP receptor activity, microbe-associated molecular pattern receptor activity, pathogen associated molecular pattern receptor activity, macrophage receptor activity, signaling pattern recognition receptor activity Definition: Combining with a pathogen-associated molecular pattern (PAMP), a structure conserved among microbial species to initiate an innate immune response. Subtypes: polysaccharide immune receptor activity [GO:0001873], lipopolysaccharide immune receptor activity [GO:0001875], GO:0001877, GO:0016019, lipoteichoic acid immune receptor activity [GO:0070892]